heparan sulfate 6-sulfotransferase activity [GO:0017095] (molecular function) Also known as: heparan sulfate 6-O-sulfotransferase activity, heparan sulphate 6-O-sulphotransferase activity, heparin 6-O-sulfotransferase activity Relationships: is a type of GO:0034483 Definition: Catalysis of the reaction: alpha-D-glucosaminyl-[heparan sulfate](n) + 3'-phosphoadenylyl sulfate = 6-sulfo-alpha-D-glucosaminyl-[heparan sulfate](n) + adenosine 3',5'-bisphosphate + H+. References: PMID:8631808 Sources: RHEA:56604